{
  "gene_symbol": "KLHL36",
  "gene": "UniProtKB:Q8N4N3",
  "term_id": "GO:0097602",
  "term_label": "cullin family protein binding",
  "gene_name": "Kelch-like protein 36"
}